{
  "gene": "UniProtKB:Q8NEY1",
  "gene_name": "Neuron navigator 1",
  "term_label": "microtubule bundle formation",
  "gene_symbol": "NAV1",
  "term_id": "GO:0001578"
}